{
  "gene_name": "Betaine--homocysteine S-methyltransferase 1",
  "gene": "UniProtKB:Q93088",
  "gene_symbol": "BHMT",
  "term_label": "betaine-homocysteine S-methyltransferase activity",
  "term_id": "GO:0047150"
}